FAD diphosphatase activity [GO:0047884] (molecular function) Relationships: is a type of GO:0004551 Definition: Catalysis of the reaction: FAD + H2O = AMP + FMN. Also known as: FAD pyrophosphatase activity, FAD pyrophosphohydrolase activity, FAD nucleotidohydrolase activity, flavin adenine dinucleotide pyrophosphatase activity, flavine adenine dinucleotide pyrophosphatase activity, riboflavin adenine dinucleotide pyrophosphatase activity, riboflavine adenine dinucleotide pyrophosphatase activity Sources: RHEA:13889